{
  "term_id": "GO:0007018",
  "gene": "UniProtKB:Q8N4N8",
  "gene_symbol": "KIF2B",
  "gene_name": "Kinesin-like protein KIF2B",
  "term_label": "microtubule-based movement"
}